ameloblast differentiation [GO:0036305] (biological process) Definition: The process in which a relatively unspecialized cell acquires specialized features of an ameloblast, a cylindrical epithelial cell in the innermost layer of the enamel organ. Sources: CL:0000059 Relationships: is a type of columnar/cuboidal epithelial cell differentiation [GO:0002065]